peptide modification [GO:0031179] (BP) Definition: The covalent alteration of one or more amino acid residues within a peptide, resulting in a change in the properties of that peptide. Relationships: is a type of peptide metabolic process [GO:0006518] Sources: GOC:mah Subtypes: GO:0001519